{
  "gene_name": "Ventricular zone-expressed PH domain-containing protein homolog 1",
  "term_label": "plasma membrane",
  "gene_symbol": "VEPH1",
  "term_id": "GO:0005886",
  "gene": "UniProtKB:Q14D04"
}